{
  "term_label": "'de novo' AMP biosynthetic process",
  "term_id": "GO:0044208",
  "gene_symbol": "ADSS2",
  "gene": "UniProtKB:P30520",
  "gene_name": "Adenylosuccinate synthetase isozyme 2"
}